{
  "gene_symbol": "RPL37AP8",
  "term_id": "UNKNOWN:0002",
  "gene": "UniProtKB:A6NKH3",
  "term_label": "Unknown biological process",
  "gene_name": "Putative ribosomal protein eL43-like"
}